receptor ligand activity [GO:0048018] (molecular function) Regulation: negatively regulated by receptor ligand inhibitor activity [GO:0141069] Sources: GOC:kv, GOC:molecular_function_refactoring, GOC:pdt Definition: The activity of a gene product that interacts with a receptor to effect a change in the activity of the receptor. Ligands may be produced by the same cell that expresses the receptor. Ligands may also be expressed at the plasma membrane of an adjacent cell (e.g. Notch ligands) or be secreted and diffuse extracellularly from their point of origin to the receiving cell (e.g. interleukins). Also known as: agonist, signaling molecule, signaling receptor ligand activity, receptor agonist activity Relationships: is a type of signaling receptor binding [GO:0005102]; is a type of GO:0030546; is part of signal transduction [GO:0007165] Subtypes: opioid peptide activity [GO:0001515], cytokine activity [GO:0005125], hormone activity [GO:0005179], GO:0005186, growth factor activity [GO:0008083], morphogen activity [GO:0016015], death receptor agonist activity [GO:0038177], chemoattractant activity [GO:0042056], chemorepellent activity [GO:0045499], pathogen-derived receptor ligand activity [GO:0140295], neuropeptide activity [GO:0160041]